{
  "term_id": "GO:0048240",
  "gene_symbol": "CATSPER3",
  "gene_name": "Cation channel sperm-associated protein 3",
  "term_label": "sperm capacitation",
  "gene": "UniProtKB:Q86XQ3"
}